{
  "term_label": "regulation of transcription by RNA polymerase II",
  "term_id": "GO:0006357",
  "gene_name": "Peregrin",
  "gene_symbol": "BRPF1",
  "gene": "UniProtKB:P55201"
}